{
  "gene": "UniProtKB:O43745",
  "gene_symbol": "CHP2",
  "term_id": "GO:0005886",
  "term_label": "plasma membrane",
  "gene_name": "Calcineurin B homologous protein 2"
}